{
  "gene_symbol": "MPP2",
  "gene": "UniProtKB:Q14168",
  "gene_name": "MAGUK p55 subfamily member 2",
  "term_id": "UNKNOWN:0001",
  "term_label": "Unknown molecular function"
}